{
  "gene_name": "Uncharacterized protein C2orf15",
  "gene_symbol": "C2orf15",
  "term_id": "UNKNOWN:0002",
  "term_label": "Unknown biological process",
  "gene": "UniProtKB:Q8WU43"
}